response to fluid shear stress [GO:0034405] (BP) Definition: Any process that results in a change in state or activity of a cell or an organism (in terms of movement, secretion, enzyme production, gene expression, etc.) as a result of a fluid shear stress stimulus. Fluid shear stress is the force acting on an object in a system where the fluid is moving across a solid surface. Sources: GOC:sl Relationships: is a type of response to stress [GO:0006950] Subtypes: response to laminar fluid shear stress [GO:0034616], cellular response to fluid shear stress [GO:0071498], response to pulsatile fluid shear stress [GO:0097701], response to oscillatory fluid shear stress [GO:0097702]